{
  "gene": "UniProtKB:Q9BV44",
  "gene_name": "tRNA (guanine(6)-N2)-methyltransferase THUMP3",
  "gene_symbol": "THUMPD3",
  "term_label": "tRNA methylation",
  "term_id": "GO:0030488"
}